{
  "gene": "UniProtKB:O60220",
  "term_label": "Unknown biological process",
  "gene_name": "Mitochondrial import inner membrane translocase subunit Tim8 A",
  "term_id": "UNKNOWN:0002",
  "gene_symbol": "TIMM8A"
}